(+)-camphor biosynthetic process [GO:0046211] (biological process) Also known as: (+)-camphor anabolism, (+)-camphor biosynthesis, (+)-camphor formation, (+)-camphor synthesis Relationships: is a type of GO:0016099; is_a GO:0042181; has part (+)-borneol dehydrogenase activity [GO:0047500]; has part geranyl-diphosphate cyclase activity [GO:0047926]; has part monoterpenyl-diphosphatase activity [GO:0050108] References: PMID:42357 Sources: GOC:ai Definition: The chemical reactions and pathways resulting in the formation of (+)-camphor, a bicyclic monoterpene ketone. Consists of the three reactions: (2E)-geranyl diphosphate = (2S,4R)-bornyl diphosphate, which is converted to (1R,2S,4R)-borneol + diphosphate, and then to (1R,4R)-camphor.